{
  "gene": "UniProtKB:Q8TF08",
  "term_label": "Unknown biological process",
  "gene_name": "Cytochrome c oxidase subunit 7B2, mitochondrial",
  "gene_symbol": "COX7B2",
  "term_id": "UNKNOWN:0002"
}